{
  "gene": "UniProtKB:Q9P219",
  "term_id": "GO:0030705",
  "gene_name": "Protein Daple",
  "gene_symbol": "CCDC88C",
  "term_label": "cytoskeleton-dependent intracellular transport"
}